{
  "gene": "UniProtKB:A0A0B4J1V0",
  "term_label": "immunoglobulin mediated immune response",
  "gene_name": "Immunoglobulin heavy variable 3-15",
  "gene_symbol": "IGHV3-15",
  "term_id": "GO:0016064"
}